{
  "gene_symbol": "WNT8A",
  "term_label": "cell fate commitment",
  "gene_name": "Protein Wnt-8a",
  "gene": "UniProtKB:Q9H1J5",
  "term_id": "GO:0045165"
}